{
  "term_label": "negative regulation of inflammatory response",
  "gene": "UniProtKB:Q96RI1",
  "gene_symbol": "NR1H4",
  "term_id": "GO:0050728",
  "gene_name": "Bile acid receptor"
}